counting factor complex [GO:0140451] (CC) Definition: A secreted multiprotein complex composed of 4 proteins, regulating group size during aggregation in cooperative development. An example of this complex is found in Dictyostelium discoideum. References: PMID:10444594, PMID:12117815, PMID:12912898, PMID:16963635, PMID:18426773 Relationships: is a type of protein-containing complex [GO:0032991]